{
  "gene_name": "POU domain class 2-associating factor 1",
  "gene_symbol": "POU2AF1",
  "term_id": "GO:0090575",
  "term_label": "RNA polymerase II transcription regulator complex",
  "gene": "UniProtKB:Q16633"
}